kinetochore disassembly involved in meiotic chromosome organization [GO:0106213] (biological process) References: PMID:27611693 Sources: GOC:mah Relationships: is a type of GO:0070192 Definition: The cell cycle process in which outer kinetochore components delocalize from the centromere, contributing to the rearrangement of chromosomes into the orientation characteristic of meiotic prophase I. Also known as: kinetochore disassembly from spindle pole body involved in chromosome organization involved in meiotic cell cycle